{
  "gene": "UniProtKB:Q9UI09",
  "gene_symbol": "NDUFA12",
  "gene_name": "NADH dehydrogenase [ubiquinone] 1 alpha subcomplex subunit 12",
  "term_label": "Unknown biological process",
  "term_id": "UNKNOWN:0002"
}